3'-flap endonuclease activity [GO:0048257] (molecular function) Definition: Catalysis of the cleavage of a 3' flap structure in DNA, but not other DNA structures; processes the 3' ends of Okazaki fragments in lagging strand DNA synthesis. References: PMID:10635319 Sources: GOC:jid Also known as: 3' flap endonuclease activity Relationships: is a type of DNA endonuclease activity, producing 3'-phosphomonoesters [GO:0016889]; is a type of flap endonuclease activity [GO:0048256]